{
  "gene_name": "Integrin alpha-D",
  "gene": "UniProtKB:Q13349",
  "gene_symbol": "ITGAD",
  "term_label": "integrin-mediated signaling pathway",
  "term_id": "GO:0007229"
}